{
  "term_label": "Unknown molecular function",
  "gene_symbol": "TMEM231",
  "gene": "UniProtKB:Q9H6L2",
  "term_id": "UNKNOWN:0001",
  "gene_name": "Transmembrane protein 231"
}